{
  "term_id": "GO:0009887",
  "gene_name": "Homeobox protein Meis3",
  "gene": "UniProtKB:Q99687",
  "term_label": "animal organ morphogenesis",
  "gene_symbol": "MEIS3"
}